peptide binding [GO:0042277] (molecular function) Relationships: is a type of binding [GO:0005488] Definition: Binding to a peptide, an organic compound comprising two or more amino acids linked by peptide bonds. Sources: GOC:jl Subtypes: amyloid-beta binding [GO:0001540], signal sequence binding [GO:0005048], peptide antigen binding [GO:0042605], GO:0042923